{
  "gene_symbol": "FAM210B",
  "gene_name": "Protein FAM210B, mitochondrial",
  "term_id": "UNKNOWN:0001",
  "gene": "UniProtKB:Q96KR6",
  "term_label": "Unknown molecular function"
}